{
  "term_id": "GO:0005737",
  "gene_symbol": "TRMT12",
  "gene": "UniProtKB:Q53H54",
  "term_label": "cytoplasm",
  "gene_name": "tRNA wybutosine-synthesizing protein 2 homolog"
}